{
  "term_id": "UNKNOWN:0002",
  "gene_name": "Purine nucleoside phosphorylase",
  "gene": "UniProtKB:P00491",
  "gene_symbol": "PNP",
  "term_label": "Unknown biological process"
}